{
  "gene_name": "Spermatogenesis- and oogenesis-specific basic helix-loop-helix-containing protein 2",
  "term_label": "RNA polymerase II cis-regulatory region sequence-specific DNA binding",
  "gene_symbol": "SOHLH2",
  "term_id": "GO:0000978",
  "gene": "UniProtKB:Q9NX45"
}